{
  "term_label": "metalloendopeptidase activity",
  "gene_symbol": "ADAM23",
  "gene_name": "Disintegrin and metalloproteinase domain-containing protein 23",
  "term_id": "GO:0004222",
  "gene": "UniProtKB:O75077"
}